{
  "gene": "UniProtKB:Q01718",
  "term_id": "GO:0005886",
  "term_label": "plasma membrane",
  "gene_symbol": "MC2R",
  "gene_name": "Adrenocorticotropic hormone receptor"
}